{
  "gene_symbol": "KDELR2",
  "term_id": "GO:0005801",
  "term_label": "cis-Golgi network",
  "gene": "UniProtKB:P33947",
  "gene_name": "ER lumen protein-retaining receptor 2"
}